venom-mediated disruption of anatomical structure in another organism [GO:0140138] (biological process) Definition: A process by which an organism effects a change that impairs the structure or function of an anatomical structure in another organism via the action of a venom. Venoms are injected into the prey by a bite or a sting. Sources: GOC:pg Relationships: is_a GO:0141060 Subtypes: venom-mediated disruption of cell wall in another organism [GO:0044278], venom-mediated pore formation in membrane of another organism [GO:0044471], venom-mediated muscle damage in another organism [GO:0044521], GO:0044523, GO:0141123